tryptophan binding [GO:0120284] (molecular function) Definition: Binding to 2-amino-3-(1H-indol-3-yl)propanoic acid. Sources: GOC:krc Relationships: is a type of amino acid binding [GO:0016597]; is a type of GO:0031406; is a type of cation binding [GO:0043169]; is a type of heterocyclic compound binding [GO:1901363] Also known as: Trp binding